{
  "gene": "UniProtKB:Q16609",
  "term_id": "UNKNOWN:0003",
  "term_label": "Unknown cellular component",
  "gene_symbol": "LPAL2",
  "gene_name": "Putative apolipoprotein(a)-like protein 2"
}